cadaverine aminopropyltransferase activity [GO:0043918] (molecular function) Also known as: cadaverine aminopropyl transferase activity Relationships: is_a GO:0016765 References: PMID:17545282 Sources: RHEA:33387 Definition: Catalysis of the reaction: cadaverine + S-adenosyl 3-(methylsulfanyl)propylamine = aminopropylcadaverine + H+ + S-methyl-5'-thioadenosine.